{
  "term_label": "RNA polymerase II cis-regulatory region sequence-specific DNA binding",
  "gene_name": "Homeobox protein EMX1",
  "gene": "UniProtKB:Q04741",
  "term_id": "GO:0000978",
  "gene_symbol": "EMX1"
}